{
  "term_id": "GO:0007218",
  "term_label": "neuropeptide signaling pathway",
  "gene_symbol": "RXFP3",
  "gene_name": "Relaxin-3 receptor 1",
  "gene": "UniProtKB:Q9NSD7"
}